recycling endosome membrane [GO:0055038] (cellular component) Definition: The lipid bilayer surrounding a recycling endosome. References: PMID:10930469, PMID:15601896, PMID:16246101 Sources: GOC:jid, GOC:rph Relationships: is a type of GO:0010008; is part of GO:0055037